{
  "term_label": "cilium",
  "gene_symbol": "IFT74",
  "term_id": "GO:0005929",
  "gene_name": "Intraflagellar transport protein 74 homolog",
  "gene": "UniProtKB:Q96LB3"
}